ventral tegmental area development [GO:1904866] (biological process) References: PMID:26548362 Sources: GOC:PARL, GOC:TermGenie, GOC:bf, GO_REF:0000094 Definition: The process whose specific outcome is the progression of a ventral tegmental area (VTA) over time, from its formation to the mature structure. Relationships: is a type of anatomical structure development [GO:0048856]; is part of GO:0030901 Also known as: VTA development, a10a development, ventral tegmental area of tsai development, ventral tegmental nucleus (tsai) development, ventral tegmental nucleus of tsai development, ventral tegmentum development, area tegmentalis ventralis (Tsai) development, area tegmentalis ventralis development, tegmentum ventrale development, ventral brain stem development, ventral tegmental area (Tsai) development, ventral tegmental nucleus (Rioch) development, ventromedial mesencephalic tegmentum development